{
  "term_id": "GO:0120147",
  "gene_symbol": "SUMF1",
  "term_label": "formylglycine-generating oxidase activity",
  "gene": "UniProtKB:Q8NBK3",
  "gene_name": "Formylglycine-generating enzyme"
}